larval lymph gland hemopoiesis [GO:0035167] (biological process) Relationships: is a type of post-embryonic hemopoiesis [GO:0035166]; is part of larval development [GO:0002164]; is part of lymph gland development [GO:0048542] Also known as: larval lymph gland haematopoiesis, larval lymph gland haemopoiesis, larval lymph gland hematopoiesis References: PMID:12445385 Sources: GOC:bf, GOC:mtg_sensu Definition: The production of blood cells from the larval lymph gland. The lymph gland consists of three to six bilaterally paired lobes that are attached to the cardioblasts during larval stages, and it degenerates during pupal stages.